{
  "term_id": "GO:0003735",
  "gene_name": "Ubiquitin-ribosomal protein eL40 fusion protein",
  "gene_symbol": "UBA52",
  "term_label": "structural constituent of ribosome",
  "gene": "UniProtKB:P62987"
}